{
  "gene_symbol": "DTX2",
  "term_label": "Notch signaling pathway",
  "gene_name": "Probable E3 ubiquitin-protein ligase DTX2",
  "term_id": "GO:0007219",
  "gene": "UniProtKB:Q86UW9"
}